{
  "gene": "UniProtKB:Q9UHB9",
  "term_id": "GO:0005047",
  "gene_symbol": "SRP68",
  "gene_name": "Signal recognition particle subunit SRP68",
  "term_label": "signal recognition particle binding"
}